{
  "term_label": "DNA-binding transcription factor activity, RNA polymerase II-specific",
  "term_id": "GO:0000981",
  "gene": "UniProtKB:P39880",
  "gene_name": "Homeobox protein cut-like 1",
  "gene_symbol": "CUX1"
}